{
  "term_label": "erythrocyte development",
  "gene": "UniProtKB:P02100",
  "gene_symbol": "HBE1",
  "gene_name": "Hemoglobin subunit epsilon",
  "term_id": "GO:0048821"
}